{
  "term_id": "GO:0060070",
  "gene_symbol": "WNT2",
  "gene": "UniProtKB:P09544",
  "term_label": "canonical Wnt signaling pathway",
  "gene_name": "Protein Wnt-2"
}